diencephalon development [GO:0021536] (biological process) Sources: GOC:cls, GOC:dgh, GOC:dph, GOC:jid, GO_REF:0000021 Relationships: is a type of anatomical structure development [GO:0048856]; is part of GO:0030900 Definition: The process whose specific outcome is the progression of the diencephalon over time, from its formation to the mature structure. The diencephalon is the paired caudal parts of the prosencephalon from which the thalamus, hypothalamus, epithalamus and subthalamus are derived; these regions regulate autonomic, visceral and endocrine function, and process information directed to the cerebral cortex.